{
  "gene": "UniProtKB:Q99525",
  "gene_name": "Histone H4-like protein type G",
  "gene_symbol": "H4C7",
  "term_id": "GO:0030527",
  "term_label": "structural constituent of chromatin"
}